{
  "gene": "UniProtKB:Q9Y3A6",
  "term_label": "Golgi ribbon formation",
  "gene_symbol": "TMED5",
  "term_id": "GO:0090161",
  "gene_name": "Transmembrane emp24 domain-containing protein 5"
}